norsolorinic acid ketoreductase activity [GO:0140393] (MF) References: PMID:10584035, PMID:8368836 Sources: RHEA:35447 Definition: Catalysis of the reaction: (1'S)-averantin + NADP+ = norsolorinic acid + NADPH. Relationships: is a type of ketoreductase activity [GO:0045703]